{
  "term_label": "cell surface receptor signaling pathway via JAK-STAT",
  "gene_name": "Tyrosine-protein kinase JAK1",
  "term_id": "GO:0007259",
  "gene": "UniProtKB:P23458",
  "gene_symbol": "JAK1"
}